{
  "gene_name": "Uncharacterized protein C3orf22",
  "term_id": "UNKNOWN:0002",
  "gene_symbol": "C3orf22",
  "term_label": "Unknown biological process",
  "gene": "UniProtKB:Q8N5N4"
}